protoporphyrinogen IX metabolic process [GO:0046501] (biological process) Relationships: is a type of porphyrin-containing compound metabolic process [GO:0006778] Subtypes: protoporphyrinogen IX biosynthetic process [GO:0006782] Also known as: protoporphyrinogen IX metabolism Definition: The chemical reactions and pathways involving protoporphyrinogen IX, the specific substrate for the enzyme ferrochelatase, which catalyzes the insertion of iron to form protoheme. It is probably also the substrate for chlorophyll formation. Note: See also the molecular function term 'ferrochelatase activity ; GO:0004325'. Sources: ISBN:0198506732